{
  "gene_symbol": "LINC01587",
  "gene": "UniProtKB:Q99440",
  "term_id": "UNKNOWN:0002",
  "term_label": "Unknown biological process",
  "gene_name": "Uncharacterized protein encoded by LINC01587"
}